cellular response to sodium arsenite [GO:1903936] (biological process) Definition: Any process that results in a change in state or activity of a cell (in terms of movement, secretion, enzyme production, gene expression, etc.) as a result of a sodium arsenite stimulus. Relationships: is a type of GO:0071243; is a type of cellular response to salt [GO:1902075]; is a type of response to sodium arsenite [GO:1903935] References: PMID:18674524 Sources: GOC:TermGenie, GO_REF:0000071